peripheral B cell negative selection [GO:0002356] (biological process) Relationships: is a type of peripheral B cell selection [GO:0002343]; is a type of B cell negative selection [GO:0002352] Sources: GOC:jal Definition: Any process leading to negative selection of B cells in the periphery. Also known as: peripheral B lymphocyte negative selection, peripheral B-cell negative selection, peripheral B-lymphocyte negative selection